{
  "term_label": "lipid storage",
  "term_id": "GO:0019915",
  "gene_name": "Perilipin-3",
  "gene": "UniProtKB:O60664",
  "gene_symbol": "PLIN3"
}